{
  "term_label": "cytoplasm",
  "gene": "UniProtKB:Q8TBB1",
  "gene_symbol": "LNX1",
  "term_id": "GO:0005737",
  "gene_name": "E3 ubiquitin-protein ligase LNX"
}